{
  "gene_symbol": "DDX11",
  "term_label": "Unknown cellular component",
  "gene_name": "ATP-dependent DNA helicase DDX11",
  "gene": "UniProtKB:Q96FC9",
  "term_id": "UNKNOWN:0003"
}